{
  "gene_symbol": "CDC42SE1",
  "gene_name": "CDC42 small effector protein 1",
  "term_id": "UNKNOWN:0002",
  "gene": "UniProtKB:Q9NRR8",
  "term_label": "Unknown biological process"
}